{
  "term_label": "nucleus",
  "gene_name": "Endoribonuclease YbeY",
  "gene_symbol": "YBEY",
  "term_id": "GO:0005634",
  "gene": "UniProtKB:P58557"
}